{
  "term_id": "UNKNOWN:0002",
  "term_label": "Unknown biological process",
  "gene_symbol": "CITED4",
  "gene": "UniProtKB:Q96RK1",
  "gene_name": "Cbp_p300-interacting transactivator 4"
}